{
  "gene_symbol": "PTCH1",
  "gene": "UniProtKB:Q13635",
  "gene_name": "Protein patched homolog 1",
  "term_id": "GO:0008158",
  "term_label": "hedgehog receptor activity"
}